{
  "term_label": "actin filament organization",
  "gene": "UniProtKB:Q6QEF8",
  "gene_name": "Coronin-6",
  "gene_symbol": "CORO6",
  "term_id": "GO:0007015"
}